{
  "term_label": "phospholipid catabolic process",
  "term_id": "GO:0009395",
  "gene_name": "Angiopoietin-related protein 3",
  "gene": "UniProtKB:Q9Y5C1",
  "gene_symbol": "ANGPTL3"
}